{
  "gene_name": "Dual specificity protein phosphatase CDC14A",
  "gene": "UniProtKB:Q9UNH5",
  "gene_symbol": "CDC14A",
  "term_label": "spindle pole",
  "term_id": "GO:0000922"
}